{
  "term_id": "GO:0005912",
  "gene": "UniProtKB:Q9NYQ6",
  "gene_name": "Cadherin EGF LAG seven-pass G-type receptor 1",
  "gene_symbol": "CELSR1",
  "term_label": "adherens junction"
}